{
  "gene_name": "Putative adrenomedullin-5-like protein",
  "gene": "UniProtKB:C9JUS6",
  "gene_symbol": "ADM5",
  "term_label": "regulation of systemic arterial blood pressure",
  "term_id": "GO:0003073"
}